{
  "gene_symbol": "IGHV1OR15-1",
  "term_label": "Unknown cellular component",
  "term_id": "UNKNOWN:0003",
  "gene_name": "Immunoglobulin heavy variable 1_OR15-1 (non-functional) (Fragment)",
  "gene": "UniProtKB:A0A075B7D0"
}